{
  "gene": "UniProtKB:O95704",
  "term_id": "GO:0005634",
  "term_label": "nucleus",
  "gene_name": "Amyloid-beta A4 precursor protein-binding family B member 3",
  "gene_symbol": "APBB3"
}